{
  "term_id": "GO:0015016",
  "gene": "UniProtKB:Q9H3R1",
  "gene_symbol": "NDST4",
  "gene_name": "Bifunctional heparan sulfate N-deacetylase_N-sulfotransferase 4",
  "term_label": "heparan sulfate N-sulfotransferase activity"
}